glycogen biosynthetic process [GO:0005978] (biological process) Relationships: is a type of GO:0005977; is a type of glucan biosynthetic process [GO:0009250] Subtypes: GO:0160249, glycogen biosynthetic process via ADP-glucose [GO:0160250] Definition: The chemical reactions and pathways resulting in the formation of glycogen, a polydisperse, highly branched glucan composed of chains of D-glucose residues. Regulation: regulated by GO:0005979; negatively regulated by negative regulation of glycogen biosynthetic process [GO:0045719]; positively regulated by positive regulation of glycogen biosynthetic process [GO:0045725] Also known as: glycogen anabolism, glycogen biosynthesis, glycogen formation, glycogen synthesis Sources: ISBN:0198506732